{
  "gene_name": "C-C motif chemokine 18",
  "term_id": "GO:0048020",
  "gene": "UniProtKB:P55774",
  "term_label": "CCR chemokine receptor binding",
  "gene_symbol": "CCL18"
}